{
  "gene_symbol": "RBM46",
  "term_id": "UNKNOWN:0002",
  "gene": "UniProtKB:Q8TBY0",
  "gene_name": "Probable RNA-binding protein 46",
  "term_label": "Unknown biological process"
}